{
  "gene_symbol": "GALR2",
  "gene": "UniProtKB:O43603",
  "term_label": "plasma membrane",
  "term_id": "GO:0005886",
  "gene_name": "Galanin receptor type 2"
}